{
  "gene_name": "Anaphase-promoting complex subunit 4",
  "term_id": "GO:0034399",
  "term_label": "nuclear periphery",
  "gene": "UniProtKB:Q9UJX5",
  "gene_symbol": "ANAPC4"
}